negative regulation of interleukin-11 production [GO:0032694] (biological process) Definition: Any process that stops, prevents, or reduces the frequency, rate, or extent of interleukin-11 production. References: PMID:29286137 Sources: GOC:mah Also known as: down regulation of interleukin-11 production, down-regulation of interleukin-11 production, downregulation of interleukin-11 production, negative regulation of IL-11 production, inhibition of interleukin-11 production, negative regulation of interleukin-11 biosynthetic process, negative regulation of interleukin-11 secretion Relationships: is a type of negative regulation of cytokine production [GO:0001818]; is a type of regulation of interleukin-11 production [GO:0032654]; negatively regulates GO:0032614